{
  "gene_symbol": "GK2",
  "term_id": "GO:0004370",
  "gene": "UniProtKB:Q14410",
  "term_label": "glycerol kinase activity",
  "gene_name": "Glycerol kinase 2"
}